snoRNA guided rRNA 2'-O-methylation [GO:0000452] (biological process) Definition: The posttranscriptional addition of methyl groups to the 2'-oxygen atom of nucleotide residues in an rRNA molecule during ribosome biogenesis using a snoRNA guide that targets the position of methylation. Also known as: snoRNA guided rRNA 2'-O-ribose methylation Sources: GOC:curators, ISBN:1555811337 Relationships: is a type of GO:0000451